{
  "term_id": "UNKNOWN:0002",
  "gene_symbol": "FHIP2A",
  "gene": "UniProtKB:Q5W0V3",
  "gene_name": "FHF complex subunit HOOK interacting protein 2A",
  "term_label": "Unknown biological process"
}